{
  "term_label": "regulation of gene expression",
  "gene": "UniProtKB:A6NGJ6",
  "gene_symbol": "TRIM64",
  "term_id": "GO:0010468",
  "gene_name": "Tripartite motif-containing protein 64"
}